{
  "term_id": "GO:0000981",
  "gene_symbol": "ZBTB7B",
  "gene_name": "Zinc finger and BTB domain-containing protein 7B",
  "term_label": "DNA-binding transcription factor activity, RNA polymerase II-specific",
  "gene": "UniProtKB:O15156"
}